{
  "gene_symbol": "OR52K2",
  "term_id": "UNKNOWN:0002",
  "term_label": "Unknown biological process",
  "gene": "UniProtKB:Q8NGK3",
  "gene_name": "Olfactory receptor 52K2"
}